positive regulation of stomach fundus smooth muscle contraction [GO:0120069] (biological process) Definition: Any process that increases the frequency, rate or extent of any stomach fundus smooth muscle contraction. References: PMID:15890336 Sources: GOC:sl Relationships: is a type of GO:0120068; is a type of GO:1904306; positively regulates stomach fundus smooth muscle contraction [GO:0014825]